axonal spine [GO:0044308] (cellular component) Relationships: is a type of neuron spine [GO:0044309]; is part of axon [GO:0030424] Sources: NIF_Subcellular:sao18239917 Definition: A spine that originates from the axon, usually from the initial segment. Also known as: axon spine